{
  "gene_symbol": "ZNF735",
  "gene_name": "Putative zinc finger protein 735",
  "term_id": "GO:0000978",
  "term_label": "RNA polymerase II cis-regulatory region sequence-specific DNA binding",
  "gene": "UniProtKB:P0CB33"
}